{
  "term_id": "GO:0050839",
  "gene_symbol": "PCDH20",
  "gene_name": "Protocadherin-20",
  "term_label": "cell adhesion molecule binding",
  "gene": "UniProtKB:Q8N6Y1"
}